{
  "term_label": "DNA-binding transcription factor activity, RNA polymerase II-specific",
  "gene": "UniProtKB:Q01167",
  "gene_symbol": "FOXK2",
  "term_id": "GO:0000981",
  "gene_name": "Forkhead box protein K2"
}